lipoate transmembrane transporter activity [GO:0170004] (molecular function) Definition: Enables the transfer of lipoate from one side of a membrane to the other. References: PMID:20980265, PMID:25971966 Relationships: is_a transmembrane transporter activity [GO:0022857]